{
  "term_id": "GO:0016286",
  "gene_symbol": "KCNN3",
  "gene": "UniProtKB:Q9UGI6",
  "term_label": "small conductance calcium-activated potassium channel activity",
  "gene_name": "Small conductance calcium-activated potassium channel protein 3"
}